{
  "gene": "UniProtKB:Q5TYX0",
  "term_id": "GO:1990756",
  "gene_name": "PRAME family member 5",
  "term_label": "ubiquitin-like ligase-substrate adaptor activity",
  "gene_symbol": "PRAMEF5"
}